{
  "term_label": "cell migration",
  "term_id": "GO:0016477",
  "gene": "UniProtKB:Q96JQ0",
  "gene_symbol": "DCHS1",
  "gene_name": "Protocadherin-16"
}